{
  "gene_name": "Hydroxylysine kinase",
  "gene": "UniProtKB:A2RU49",
  "term_id": "UNKNOWN:0003",
  "term_label": "Unknown cellular component",
  "gene_symbol": "HYKK"
}